{
  "gene": "UniProtKB:P47871",
  "term_id": "GO:0007189",
  "gene_symbol": "GCGR",
  "term_label": "adenylate cyclase-activating G protein-coupled receptor signaling pathway",
  "gene_name": "Glucagon receptor"
}